{
  "term_id": "GO:0005634",
  "gene_name": "Zinc finger protein 334",
  "gene_symbol": "ZNF334",
  "gene": "UniProtKB:Q9HCZ1",
  "term_label": "nucleus"
}